{
  "term_id": "GO:0030574",
  "gene_symbol": "MMP15",
  "gene": "UniProtKB:P51511",
  "gene_name": "Matrix metalloproteinase-15",
  "term_label": "collagen catabolic process"
}